alpha4-beta1 integrin-CD47 complex [GO:0071120] (cellular component) Definition: A protein complex that consists of an alpha4-beta1 integrin complex bound to the cell surface antigen CD47. References: PMID:15292185 Also known as: ITGA4-ITGB1-CB47 complex Relationships: is a type of GO:0098797